{
  "term_label": "calcium ion binding",
  "gene": "UniProtKB:Q15293",
  "gene_name": "Reticulocalbin-1",
  "term_id": "GO:0005509",
  "gene_symbol": "RCN1"
}